{
  "gene_symbol": "TRPC3",
  "gene_name": "Short transient receptor potential channel 3",
  "term_id": "GO:0051480",
  "gene": "UniProtKB:Q13507",
  "term_label": "regulation of cytosolic calcium ion concentration"
}